synaptic vesicle endosomal processing [GO:0099532] (biological process) Subtypes: GO:0099592 Also known as: synaptic vesicle processing via endosome Note: This covers processing of synaptic vesicles trafficked to synapse as well as of endocytosed vesicles as part of recycling. It is there for not part of the synaptic vesicle cycle. Definition: The process in which synaptic vesicles fuse to the presynaptic endosome followed by sorting of synaptic vesicle components and budding of new synaptic vesicles. Sources: GOC:aruk, GOC:bc, GOC:dos Relationships: is a type of GO:0016197